{
  "gene": "UniProtKB:Q8TEP8",
  "term_id": "GO:0090307",
  "term_label": "mitotic spindle assembly",
  "gene_symbol": "CEP192",
  "gene_name": "Centrosomal protein of 192 kDa"
}